negative regulation of fusion cell fate specification [GO:0035157] (biological process) Also known as: down regulation of fusion cell fate specification, down-regulation of fusion cell fate specification, downregulation of fusion cell fate specification, inhibition of fusion cell fate specification Relationships: is_a GO:0009996; is a type of negative regulation of multicellular organismal process [GO:0051241]; negatively regulates fusion cell fate specification [GO:0035156] References: PMID:10684581 Definition: Any process that restricts, stops or prevents a cell from adopting a fusion cell fate. Once the terminal and fusion fates have been correctly induced, inhibitory feedback loops prevent the remaining branch cells from assuming similar fates.